{
  "term_id": "GO:0005886",
  "gene_name": "Proteinase-activated receptor 4",
  "gene": "UniProtKB:Q96RI0",
  "gene_symbol": "F2RL3",
  "term_label": "plasma membrane"
}